de novo centriole assembly [GO:0097742] (biological process) Subtypes: de novo centriole assembly via blepharoplast [GO:0097743], de novo centriole assembly involved in multi-ciliated epithelial cell differentiation [GO:0098535] Relationships: is a type of centriole assembly [GO:0098534] Definition: Centriole assembly in which a centriole arises de novo, rather than by replication from an existing centriole. This process may occur via different mechanisms. Examples include the deuterosome pathway in multicilated epithelial animal cells and formation of centrioles during parthenogenesis in some insects. Also known as: acentriolar basal body biogenesis, de novo basal body amplification, de novo basal body assembly, de novo basal body biogenesis, de novo basal body generation, de novo centriole amplification, de novo ciliary basal body assembly, multiciliation, multiciliogenesis References: PMID:25047614, PMID:25291643 Sources: GOC:cilia